{
  "gene_symbol": "LHX1",
  "term_label": "neuron differentiation",
  "term_id": "GO:0030182",
  "gene_name": "LIM_homeobox protein Lhx1",
  "gene": "UniProtKB:P48742"
}